{
  "gene": "UniProtKB:O75363",
  "gene_name": "Breast carcinoma-amplified sequence 1",
  "term_id": "UNKNOWN:0003",
  "term_label": "Unknown cellular component",
  "gene_symbol": "BCAS1"
}